{
  "term_id": "GO:0004861",
  "term_label": "cyclin-dependent protein serine/threonine kinase inhibitor activity",
  "gene_name": "Cyclin-dependent kinase 4 inhibitor C",
  "gene": "UniProtKB:P42773",
  "gene_symbol": "CDKN2C"
}